{
  "gene": "UniProtKB:Q9H1F0",
  "term_id": "GO:0019731",
  "gene_symbol": "WFDC10A",
  "gene_name": "WAP four-disulfide core domain protein 10A",
  "term_label": "antibacterial humoral response"
}